{
  "term_label": "regulation of cytokine production",
  "gene_name": "Hypermethylated in cancer 2 protein",
  "term_id": "GO:0001817",
  "gene_symbol": "HIC2",
  "gene": "UniProtKB:Q96JB3"
}